{
  "gene": "UniProtKB:Q3B7S5",
  "term_id": "UNKNOWN:0003",
  "gene_symbol": "SMIM21",
  "term_label": "Unknown cellular component",
  "gene_name": "Small integral membrane protein 21"
}